{
  "gene": "UniProtKB:Q9Y278",
  "gene_name": "Heparan sulfate glucosamine 3-O-sulfotransferase 2",
  "term_label": "Unknown cellular component",
  "gene_symbol": "HS3ST2",
  "term_id": "UNKNOWN:0003"
}